negative regulation of lymphocyte mediated immunity [GO:0002707] (biological process) Relationships: is_a negative regulation of leukocyte mediated immunity [GO:0002704]; is a type of GO:0002706; negatively regulates GO:0002449 Subtypes: negative regulation of T cell mediated immunity [GO:0002710], negative regulation of B cell mediated immunity [GO:0002713], negative regulation of natural killer cell mediated immunity [GO:0002716] Also known as: down regulation of lymphocyte mediated immunity, down-regulation of lymphocyte mediated immunity, downregulation of lymphocyte mediated immunity, inhibition of lymphocyte mediated immunity Definition: Any process that stops, prevents, or reduces the frequency, rate, or extent of lymphocyte mediated immunity. Sources: GOC:add